{
  "gene_name": "P2X purinoceptor 6",
  "term_label": "plasma membrane",
  "gene": "UniProtKB:O15547",
  "gene_symbol": "P2RX6",
  "term_id": "GO:0005886"
}